{
  "gene_name": "Putative inactive carboxylesterase 4",
  "term_label": "retinyl-palmitate esterase activity",
  "term_id": "GO:0050253",
  "gene": "UniProtKB:Q9UKY3",
  "gene_symbol": "CES1P1"
}